{
  "gene_symbol": "AIFM3",
  "term_label": "mitochondrion",
  "term_id": "GO:0005739",
  "gene": "UniProtKB:Q96NN9",
  "gene_name": "Apoptosis-inducing factor 3"
}